{
  "gene_symbol": "UVSSA",
  "gene": "UniProtKB:Q2YD98",
  "term_id": "GO:0000993",
  "gene_name": "UV-stimulated scaffold protein A",
  "term_label": "RNA polymerase II complex binding"
}